{
  "gene_symbol": "P2RY10",
  "gene": "UniProtKB:O00398",
  "gene_name": "Putative P2Y purinoceptor 10",
  "term_id": "GO:0005886",
  "term_label": "plasma membrane"
}